{
  "term_id": "GO:0006357",
  "gene_name": "Zinc finger protein 16",
  "gene_symbol": "ZNF16",
  "term_label": "regulation of transcription by RNA polymerase II",
  "gene": "UniProtKB:P17020"
}